methylquercetagetin 6-O-methyltransferase activity [GO:0030759] (MF) Relationships: is a type of S-adenosylmethionine-dependent methyltransferase activity [GO:0008757] Definition: Catalysis of the reaction: 3',4',5,6-tetrahydroxy-3,7-dimethoxyflavone + S-adenosyl-L-methionine(1+) = 3',4',5-trihydroxy-3,6,7-trimethoxyflavone + S-adenosyl-L-homocysteine + H+. Also known as: 6-OMT, S-adenosyl-L-methionine:3',4',5,6-tetrahydroxy-3,7-dimethoxyflavone 6-O-methyltransferase activity, flavonol 6-O-methyltransferase activity, flavonol 6-methyltransferase activity Sources: EC:2.1.1.84, RHEA:18717